{
  "gene_symbol": "KRTAP4-12",
  "term_label": "hair cycle",
  "gene_name": "Keratin-associated protein 4-12",
  "term_id": "GO:0042633",
  "gene": "UniProtKB:Q9BQ66"
}